{
  "gene_name": "Sarcoplasmic_endoplasmic reticulum calcium ATPase regulator DWORF",
  "gene_symbol": "STRIT1",
  "term_label": "Unknown molecular function",
  "term_id": "UNKNOWN:0001",
  "gene": "UniProtKB:P0DN84"
}